smoothened signaling pathway involved in regulation of secondary heart field cardioblast proliferation [GO:0003271] (biological process) Relationships: is_a GO:0007224; is a type of cell surface receptor signaling pathway involved in heart development [GO:0061311]; is part of GO:0003266 Sources: GOC:mtg_heart Definition: The series of molecular signals generated as a consequence of activation of the transmembrane protein Smoothened contributing to the modulation of the frequency, rate or extent of cardioblast proliferation in the secondary heart field. A cardioblast is a cardiac precursor cell. It is a cell that has been committed to a cardiac fate, but will undergo more cell division rather than terminally differentiating. Also known as: hedgehog signaling pathway involved in regulation of second heart field cardioblast proliferation, hh signaling pathway involved in regulation of second heart field cardioblast proliferation, smoothened receptor signaling pathway involved in regulation of second heart field cardioblast proliferation, smoothened receptor signaling pathway involved in regulation of secondary heart field cardioblast proliferation, smoothened receptor signalling pathway involved in regulation of secondary heart field cardioblast proliferation